{
  "gene_symbol": "KRT25",
  "term_label": "epithelial cell differentiation",
  "term_id": "GO:0030855",
  "gene": "UniProtKB:Q7Z3Z0",
  "gene_name": "Keratin, type I cytoskeletal 25"
}